transcription factor TFIIIB-beta complex [GO:0034733] (cellular component) References: PMID:11433012 Definition: A transcription factor TFIIIB-beta complex that contains the TATA-binding protein (TBP), B'' and BRF, and is involved in the regulation of transcription from type 2 RNA polymerase III promoters. Relationships: is a type of transcription factor TFIIIB complex [GO:0000126] Note: Note that the subunits of TFIIIB-beta are conserved between human and yeast; however, in yeast a single TFIIIB complex regulates transcription of tRNA, 5S rRNA and U6 snRNA genes, whereas two different TBP-dependent TFIIIB activities exist in humans.